{
  "gene_symbol": "MTG2",
  "gene": "UniProtKB:Q9H4K7",
  "term_id": "GO:0005739",
  "term_label": "mitochondrion",
  "gene_name": "Mitochondrial ribosome-associated GTPase 2"
}